{
  "gene_name": "Neurocan core protein",
  "gene_symbol": "NCAN",
  "term_id": "GO:0001501",
  "term_label": "skeletal system development",
  "gene": "UniProtKB:O14594"
}